{
  "term_id": "UNKNOWN:0002",
  "term_label": "Unknown biological process",
  "gene_name": "Putative Arf-GAP with GTPase, ANK repeat and PH domain-containing protein 7",
  "gene_symbol": "AGAP7P",
  "gene": "UniProtKB:Q5VUJ5"
}